pteridine metabolic process [GO:0019889] (biological process) Definition: The chemical reactions and pathways involving pteridine, pyrazino(2,3-dipyrimidine), the parent structure of pterins and the pteroyl group. Relationships: is a type of pteridine-containing compound metabolic process [GO:0042558] Subtypes: pteridine biosynthetic process [GO:0006728], pteridine catabolic process [GO:0019990] Also known as: pteridine metabolism Sources: GOC:go_curators, ISBN:0198506732